positive regulation of gene expression via chromosomal CpG island demethylation [GO:0044029] (biological process) Also known as: DNA demethylation, DNA hypomethylation of CpG island, hypomethylation of CpG island, positive regulation of gene expression via chromosomal CpG dinucleotide demethylation References: PMID:36150101 Sources: Wikipedia:Cpg_island Relationships: is a type of GO:0045815 Definition: An epigenetic gene regulation mechanism that positively regulates gene expression by demethylation of cytosine residues in chromosomal CpG islands. CpG islands are genomic regions that contain a high frequency of the CG dinucleotide and are often associated with the transcription start site of genes.